{
  "term_id": "GO:0000776",
  "gene_name": "Spindle and kinetochore-associated protein 3",
  "term_label": "kinetochore",
  "gene_symbol": "SKA3",
  "gene": "UniProtKB:Q8IX90"
}